cellooligosaccharide catabolic process [GO:2000903] (biological process) Definition: The chemical reactions and pathways resulting in the breakdown of a cellooligosaccharide. Sources: GOC:mengo_curators Also known as: cellooligosaccharide catabolism Relationships: is a type of oligosaccharide catabolic process [GO:0009313]; is a type of cellooligosaccharide metabolic process [GO:2000902] Regulation: regulated by regulation of cellooligosaccharide catabolic process [GO:2000963]; negatively regulated by negative regulation of cellooligosaccharide catabolic process [GO:2000964]; positively regulated by GO:2000965